{
  "gene_name": "TM2 domain-containing protein 2",
  "term_label": "Unknown cellular component",
  "gene": "UniProtKB:Q9BX73",
  "term_id": "UNKNOWN:0003",
  "gene_symbol": "TM2D2"
}